{
  "gene_symbol": "RGP1",
  "gene": "UniProtKB:Q92546",
  "term_label": "Golgi membrane",
  "gene_name": "RAB6A-GEF complex partner protein 2",
  "term_id": "GO:0000139"
}